dol-P-Man:Man(3)GlcN-acyl-PI alpha-1,2-mannosyltransferase activity [GO:0120565] (molecular function) Relationships: is a type of alpha-1,2-mannosyltransferase activity [GO:0000026]; is a type of GPI mannosyltransferase activity [GO:0004376] Definition: Catalysis of the transfer of an alpha-D-mannosyl residue from dolichol-P-mannose to Man(3)-GlcN-acyl-PI, forming an alpha-(1->2)-D-mannosyl-D-mannose linkage. This transfers a fourth mannose to the GPI precursor, which is only present in some organisms/cell types. Also known as: GPI-MT-IV activity, glycosylphosphatidylinositol-mannosyltransferase IV activity References: PMID:15208306